{
  "gene": "UniProtKB:P20810",
  "term_label": "Unknown biological process",
  "gene_symbol": "CAST",
  "term_id": "UNKNOWN:0002",
  "gene_name": "Calpastatin"
}